{
  "gene_name": "MICOS complex subunit MIC10",
  "gene_symbol": "MICOS10",
  "term_label": "Unknown biological process",
  "gene": "UniProtKB:Q5TGZ0",
  "term_id": "UNKNOWN:0002"
}